{
  "gene_name": "Speedy protein C",
  "gene_symbol": "SPDYC",
  "term_id": "UNKNOWN:0003",
  "gene": "UniProtKB:Q5MJ68",
  "term_label": "Unknown cellular component"
}